plasma membrane to endosome transport [GO:0048227] (biological process) Definition: Transport of a vesicle from the plasma membrane to the endosome. Sources: GOC:jid Relationships: is a type of GO:0016192 Subtypes: GO:0099646